{
  "term_id": "GO:0003779",
  "gene_symbol": "LRRC10",
  "term_label": "actin binding",
  "gene_name": "Leucine-rich repeat-containing protein 10",
  "gene": "UniProtKB:Q5BKY1"
}